negative regulation of shelterin complex assembly [GO:1904791] (biological process) Definition: Any process that stops, prevents or reduces the frequency, rate or extent of shelterin complex assembly. References: PMID:24270157 Sources: GOC:BHF, GOC:BHF_telomere, GOC:TermGenie, GOC:nc, GO_REF:0000058 Also known as: down regulation of Pot1 complex assembly, down regulation of Pot1-Tpz1 complex assembly, down regulation of shelterin complex formation, down regulation of telosome assembly, down-regulation of Pot1 complex assembly, down-regulation of Pot1-Tpz1 complex assembly, down-regulation of shelterin complex formation, down-regulation of telosome assembly, downregulation of Pot1 complex assembly, downregulation of Pot1-Tpz1 complex assembly, downregulation of shelterin complex formation, downregulation of telosome assembly, negative regulation of Pot1 complex assembly, negative regulation of Pot1-Tpz1 complex assembly, negative regulation of shelterin complex formation, negative regulation of telosome assembly, inhibition of Pot1 complex assembly, inhibition of Pot1-Tpz1 complex assembly, inhibition of shelterin complex formation, inhibition of telosome assembly Relationships: is a type of negative regulation of protein-containing complex assembly [GO:0031333]; is a type of regulation of shelterin complex assembly [GO:1904790]; negatively regulates GO:0071573